{
  "term_id": "GO:0052725",
  "gene": "UniProtKB:Q13572",
  "gene_name": "Inositol-tetrakisphosphate 1-kinase",
  "term_label": "inositol-1,3,4-trisphosphate 6-kinase activity",
  "gene_symbol": "ITPK1"
}